perinuclear endoplasmic reticulum [GO:0097038] (CC) Definition: The portion of endoplasmic reticulum, the intracellular network of tubules and cisternae, that occurs near the nucleus. The lumen of the perinuclear endoplasmic reticulum is contiguous with the nuclear envelope lumen (also called perinuclear space), the region between the inner and outer nuclear membranes. Sources: GOC:bf, GOC:mah, GOC:mcc, GOC:pr, GOC:vw Also known as: perinuclear ER Relationships: is a type of cellular anatomical structure [GO:0110165]; is part of endoplasmic reticulum [GO:0005783]; is part of perinuclear region of cytoplasm [GO:0048471]